{
  "gene_symbol": "AKTIP",
  "term_label": "DNA damage tolerance",
  "gene": "UniProtKB:Q9H8T0",
  "gene_name": "AKT-interacting protein",
  "term_id": "GO:0006301"
}